{
  "term_id": "UNKNOWN:0003",
  "gene": "UniProtKB:Q9UGB7",
  "gene_name": "Inositol oxygenase",
  "term_label": "Unknown cellular component",
  "gene_symbol": "MIOX"
}